{
  "gene_name": "Testis-specific gene 10 protein",
  "term_label": "Unknown molecular function",
  "gene_symbol": "TSGA10",
  "gene": "UniProtKB:Q9BZW7",
  "term_id": "UNKNOWN:0001"
}